{
  "gene": "UniProtKB:Q9UH03",
  "gene_symbol": "SEPTIN3",
  "gene_name": "Neuronal-specific septin-3",
  "term_id": "GO:0061640",
  "term_label": "cytoskeleton-dependent cytokinesis"
}